alpha-ketoacid dehydrogenase complex [GO:0045240] (cellular component) Definition: A multi-enzyme complex that catalyzes the oxidative decarboxylation of an alpha-ketoacid - pyruvate, a branched-chain alpha-ketoacid or alpha-ketoglutarate (also known as 2-oxoglutarate). The complex comprises multiple copies of three enzymes referred to as E1, E2 and E3: a dihydrolipoyl transacylase (E2) forms the core of the complex, with an alpha-ketoacid dehydrogenase (E1) and a dihydrolipoamide dehydrogenase (E3) attached through non-covalent bonds. The E1 and E2 components are specific to different alpha-ketoacid dehydrogenase complexes, whereas the E3 component is the same. Additional proteins may also be present. References: PMID:10745006 Sources: GOC:mah Also known as: 2-oxoacid dehydrogenase complex, dihydrolipoyl dehydrogenase complex Relationships: is a type of GO:1990204 Subtypes: oxoglutarate dehydrogenase complex [GO:0045252], GO:0045254, branched-chain alpha-ketoacid dehydrogenase complex [GO:0160157], GO:0160167